{
  "gene": "UniProtKB:O15020",
  "term_id": "GO:0042995",
  "gene_symbol": "SPTBN2",
  "term_label": "cell projection",
  "gene_name": "Spectrin beta chain, non-erythrocytic 2"
}